{
  "gene_name": "Ras-related protein Rab-5C",
  "gene": "UniProtKB:P51148",
  "term_id": "GO:0006897",
  "gene_symbol": "RAB5C",
  "term_label": "endocytosis"
}